{
  "term_label": "Unknown cellular component",
  "gene_name": "Recombining binding protein suppressor of hairless-like protein",
  "gene": "UniProtKB:Q9UBG7",
  "gene_symbol": "RBPJL",
  "term_id": "UNKNOWN:0003"
}